{
  "term_id": "GO:0043123",
  "gene": "UniProtKB:Q8IV45",
  "term_label": "positive regulation of canonical NF-kappaB signal transduction",
  "gene_symbol": "UNC5CL",
  "gene_name": "UNC5C-like protein"
}